{
  "gene_name": "Small ribosomal subunit protein uS2B",
  "term_id": "GO:0002181",
  "term_label": "cytoplasmic translation",
  "gene": "UniProtKB:A0A8I5KQE6",
  "gene_symbol": "RPSA2"
}